{
  "term_label": "regulation of immune system process",
  "gene_name": "B-cell CLL_lymphoma 6 member B protein",
  "gene": "UniProtKB:Q8N143",
  "gene_symbol": "BCL6B",
  "term_id": "GO:0002682"
}